{
  "gene": "UniProtKB:Q9P1G2",
  "gene_symbol": "RBM12B-AS1",
  "term_label": "Unknown biological process",
  "gene_name": "Putative uncharacterized protein encoded by RBM12B-AS1",
  "term_id": "UNKNOWN:0002"
}